{
  "term_label": "vesicle-mediated transport",
  "gene": "UniProtKB:Q9UPP2",
  "gene_name": "IQ motif and SEC7 domain-containing protein 3",
  "term_id": "GO:0016192",
  "gene_symbol": "IQSEC3"
}